{
  "gene_name": "Myc proto-oncogene protein",
  "gene_symbol": "MYC",
  "term_label": "regulation of transcription by RNA polymerase II",
  "gene": "UniProtKB:P01106",
  "term_id": "GO:0006357"
}